{
  "gene_name": "Homeobox protein Hox-C13",
  "term_label": "regulation of transcription by RNA polymerase II",
  "gene_symbol": "HOXC13",
  "gene": "UniProtKB:P31276",
  "term_id": "GO:0006357"
}